{
  "gene_name": "Protein TALPID3",
  "term_label": "Unknown molecular function",
  "term_id": "UNKNOWN:0001",
  "gene_symbol": "KIAA0586",
  "gene": "UniProtKB:Q9BVV6"
}